{
  "gene_name": "Protein-tyrosine sulfotransferase 1",
  "gene": "UniProtKB:O60507",
  "term_id": "GO:0008476",
  "term_label": "protein-tyrosine sulfotransferase activity",
  "gene_symbol": "TPST1"
}